{
  "gene_name": "Muscarinic acetylcholine receptor M3",
  "term_id": "GO:0006940",
  "gene_symbol": "CHRM3",
  "term_label": "regulation of smooth muscle contraction",
  "gene": "UniProtKB:P20309"
}